actin cytoskeleton-regulatory complex [GO:1990964] (cellular component) Relationships: is a type of GO:0032991 Note: An example of this is Pan1 in Saccharomyces cerevisiae (UniProt ID P32521) in PMID:10594004 (inferred from direct assay). Definition: A protein complex probably required for the internalization of endosomes during actin-coupled endocytosis. Links the site of endocytosis to the cell membrane-associated actin cytoskeleton, coordinating ARP2/3 stimulation at the later stages of endocytosis. Present in the late endocytic coat. References: PMID:10594004, PMID:11739778 Sources: GOC:bhm